{
  "gene": "UniProtKB:Q8N6L0",
  "gene_symbol": "KASH5",
  "gene_name": "Protein KASH5",
  "term_label": "spindle assembly",
  "term_id": "GO:0051225"
}